{
  "gene": "UniProtKB:Q9BXY4",
  "gene_name": "R-spondin-3",
  "gene_symbol": "RSPO3",
  "term_id": "GO:0090263",
  "term_label": "positive regulation of canonical Wnt signaling pathway"
}